{
  "gene_name": "Inactive ubiquitin carboxyl-terminal hydrolase 17-like protein 7",
  "term_id": "GO:0005829",
  "gene_symbol": "USP17L7",
  "term_label": "cytosol",
  "gene": "UniProtKB:P0C7H9"
}